{
  "term_label": "centrosome",
  "gene_name": "Centrosomal protein of 135 kDa",
  "term_id": "GO:0005813",
  "gene_symbol": "CEP135",
  "gene": "UniProtKB:Q66GS9"
}